{
  "term_id": "UNKNOWN:0001",
  "gene_name": "Armadillo repeat-containing X-linked protein 4",
  "term_label": "Unknown molecular function",
  "gene_symbol": "ARMCX4",
  "gene": "UniProtKB:Q5H9R4"
}